dihydropyrimidine dehydrogenase (NAD+) activity [GO:0004159] (molecular function) Definition: Catalysis of the reaction: a 5,6-dihydropyrimidine (5,6-dihydrouracil or 5,6-dihydrothymine) + NAD+ = a pyrimidine (uracil or thymine) + NADH + H+. References: PMID:23150645 Also known as: dihydrothymine dehydrogenase (NAD+) activity, dihydrouracil dehydrogenase (NAD+) activity, thymine reductase activity, uracil reductase activity, 5,6-dihydrouracil:NAD+ oxidoreductase activity, pyrimidine reductase activity Relationships: is a type of oxidoreductase activity, acting on the CH-CH group of donors, NAD or NADP as acceptor [GO:0016628]